tissue regeneration [GO:0042246] (biological process) Definition: The regrowth of lost or destroyed tissues. Sources: GOC:curators Subtypes: fin regeneration [GO:0031101], skeletal muscle tissue regeneration [GO:0043403], GO:0061026, GO:0097719, GO:1990399, bone regeneration [GO:1990523] Relationships: is a type of GO:0031099; is_a GO:0048589